regulation of heat dissipation [GO:0031654] (biological process) Relationships: is a type of regulation of multicellular organismal process [GO:0051239]; regulates heat dissipation [GO:0031653] Sources: GOC:dph, GOC:mah, GOC:tb Definition: Any process that modulates the rate or extent of heat dissipation. Subtypes: negative regulation of heat dissipation [GO:0031655], GO:0031656